{
  "term_id": "UNKNOWN:0003",
  "gene_name": "Uncharacterized protein C19orf84",
  "gene": "UniProtKB:I3L1E1",
  "gene_symbol": "C19orf84",
  "term_label": "Unknown cellular component"
}